{
  "term_label": "Unknown cellular component",
  "gene": "UniProtKB:Q9BZ29",
  "gene_name": "Dedicator of cytokinesis protein 9",
  "term_id": "UNKNOWN:0003",
  "gene_symbol": "DOCK9"
}